{
  "term_label": "chloride channel activity",
  "gene_symbol": "GABRA2",
  "gene": "UniProtKB:P47869",
  "gene_name": "Gamma-aminobutyric acid receptor subunit alpha-2",
  "term_id": "GO:0005254"
}